{
  "gene": "UniProtKB:P0DME0",
  "term_id": "UNKNOWN:0002",
  "gene_name": "Protein SETSIP",
  "term_label": "Unknown biological process",
  "gene_symbol": "SETSIP"
}